{
  "gene_symbol": "SBNO1",
  "gene_name": "Protein strawberry notch homolog 1",
  "term_label": "nucleus",
  "term_id": "GO:0005634",
  "gene": "UniProtKB:A3KN83"
}